{
  "gene": "UniProtKB:Q9UBL9",
  "gene_symbol": "P2RX2",
  "term_id": "GO:0070588",
  "gene_name": "P2X purinoceptor 2",
  "term_label": "calcium ion transmembrane transport"
}